{
  "term_id": "GO:0005634",
  "gene_symbol": "MT1E",
  "term_label": "nucleus",
  "gene_name": "Metallothionein-1E",
  "gene": "UniProtKB:P04732"
}